{
  "gene_name": "Lysine-rich nucleolar protein 1",
  "term_id": "UNKNOWN:0002",
  "term_label": "Unknown biological process",
  "gene_symbol": "KNOP1",
  "gene": "UniProtKB:Q1ED39"
}